myxococcal fruiting body development [GO:0030583] (biological process) Relationships: is a type of developmental process [GO:0032502]; is a type of response to starvation [GO:0042594] References: PMID:11121786 Sources: GOC:mtg_sensu, ISBN:0815316194 Note: For example, as seen in myxobacterium. It is not intended to describe fruiting body development as is Dictyostelium. Definition: The process whose specific outcome is the progression of the myxococcal fruiting body over time, from its formation to the mature structure. The process begins when myxococci respond to a lack of nutrients in the environment and ends when the myxococcal fruiting body is a mature structure. Also known as: fruiting body development in cellular response to starvation, fruiting body development in response to starvation